interleukin-13 production [GO:0032616] (biological process) Definition: The appearance of interleukin-13 due to biosynthesis or secretion following a cellular stimulus, resulting in an increase in its intracellular or extracellular levels. Regulation: regulated by regulation of interleukin-13 production [GO:0032656]; RO_0002212 by negative regulation of interleukin-13 production [GO:0032696]; positively regulated by positive regulation of interleukin-13 production [GO:0032736] Sources: GOC:mah Relationships: is a type of cytokine production [GO:0001816] Also known as: IL-13 production, interleukin-13 biosynthetic process, interleukin-13 secretion